{
  "gene_symbol": "TRGV9",
  "gene": "UniProtKB:Q99603",
  "term_label": "external side of plasma membrane",
  "term_id": "GO:0009897",
  "gene_name": "T cell receptor gamma variable 9"
}